stamen filament development [GO:0080086] (biological process) Also known as: filament development Definition: The process whose specific outcome is the progression of the filament over time, from its formation to the mature structure. Filament is the stalk of a stamen. Relationships: is a type of GO:0003006; is a type of GO:0048856; is part of stamen development [GO:0048443] References: PMID:19139039 Sources: PO:0009067